desmosome [GO:0030057] (cellular component) Sources: GOC:mah, GOC:mtg_muscle, ISBN:0815332181 Also known as: macula adherens, spot desmosome Relationships: is a type of cell-cell junction [GO:0005911] Definition: A cell-cell junction in which: on the cytoplasmic surface of each interacting plasma membrane is a dense plaque composed of a mixture of intracellular anchor proteins; a bundle of keratin intermediate filaments is attached to the surface of each plaque; transmembrane adhesion proteins of the cadherin family bind to the plaques and interact through their extracellular domains to hold the adjacent membranes together by a Ca2+-dependent mechanism.